glucan endo-1,3-beta-D-glucosidase activity [GO:0042973] (molecular function) Also known as: beta-1,3-glucanase, endo-(1,3)-beta-D-glucanase activity, endo-(1->3)-beta-D-glucanase activity, endo-1,3-beta-D-glucanase, endo-1,3-beta-glucanase activity, endo-1,3-beta-glucosidase activity, laminaranase activity, laminarinase activity, (1->3)-beta-glucan 3-glucanohydrolase activity, (1->3)-beta-glucan endohydrolase activity, 1,3-beta-D-glucan 3-glucanohydrolase activity, 1,3-beta-D-glucan glucanohydrolase activity, callase activity, kitalase activity, oligo-1,3-glucosidase activity Definition: Catalysis of the hydrolysis of (1->3)-beta-D-glucosidic linkages in (1->3)-beta-D-glucans. Sources: EC:3.2.1.39 Relationships: is a type of GO:0008422